mugineic-acid 3-dioxygenase activity [GO:0033761] (molecular function) Sources: EC:1.14.11.25 Also known as: IDS2, mugineic acid,2-oxoglutarate:oxygen oxidoreductase (3-hydroxylating) activity Definition: Catalysis of the reaction: mugineate + 2-oxoglutarate + O2 = 3-epihydroxymugineate + CO2 + H+ + succinate. Also converts 2'-deoxymugineate to 3-epihydroxy-2'-deoxymugineate. Relationships: is a type of 2-oxoglutarate-dependent dioxygenase activity [GO:0016706]